{
  "term_id": "GO:0004984",
  "gene_name": "Olfactory receptor 2A7",
  "gene": "UniProtKB:Q96R45",
  "gene_symbol": "OR2A7",
  "term_label": "olfactory receptor activity"
}